{
  "term_id": "UNKNOWN:0001",
  "gene_symbol": "NLRP4",
  "gene_name": "NACHT, LRR and PYD domains-containing protein 4",
  "gene": "UniProtKB:Q96MN2",
  "term_label": "Unknown molecular function"
}